{
  "gene_symbol": "CHRNB1",
  "gene": "UniProtKB:P11230",
  "term_id": "GO:0003009",
  "gene_name": "Acetylcholine receptor subunit beta",
  "term_label": "skeletal muscle contraction"
}